{
  "term_id": "GO:0016339",
  "gene": "UniProtKB:P33151",
  "gene_symbol": "CDH5",
  "term_label": "calcium-dependent cell-cell adhesion",
  "gene_name": "Cadherin-5"
}